{
  "gene": "UniProtKB:P53677",
  "term_id": "GO:0005802",
  "term_label": "trans-Golgi network",
  "gene_symbol": "AP3M2",
  "gene_name": "AP-3 complex subunit mu-2"
}